regulation of sensory perception of bitter taste [GO:1904660] (biological process) Subtypes: negative regulation of sensory perception of bitter taste [GO:1904661], GO:1904662 Relationships: is a type of regulation of sensory perception [GO:0051931]; regulates sensory perception of bitter taste [GO:0050913] Definition: Any process that modulates the frequency, rate or extent of sensory perception of bitter taste. References: PMID:1716172 Sources: GOC:TermGenie, GOC:mr, GO_REF:0000058 Also known as: regulation of bitter taste perception